{
  "gene": "UniProtKB:P23919",
  "gene_symbol": "DTYMK",
  "term_label": "nucleus",
  "term_id": "GO:0005634",
  "gene_name": "Thymidylate kinase"
}